cyclic nucleotide catabolic process [GO:0009214] (biological process) Regulation: regulated by GO:0030805 Subtypes: cAMP catabolic process [GO:0006198], cGMP catabolic process [GO:0046069] Also known as: cyclic nucleotide breakdown, cyclic nucleotide catabolism, cyclic nucleotide degradation Definition: The chemical reactions and pathways resulting in the breakdown of a cyclic nucleotide, a nucleotide in which the phosphate group is in diester linkage to two positions on the sugar residue. Sources: GOC:go_curators, ISBN:0198506732 Relationships: is a type of GO:0009166; is a type of GO:0009187